{
  "term_label": "transforming growth factor beta binding",
  "gene": "UniProtKB:Q14392",
  "term_id": "GO:0050431",
  "gene_symbol": "LRRC32",
  "gene_name": "Transforming growth factor beta activator LRRC32"
}